{
  "gene_symbol": "RTL6",
  "gene": "UniProtKB:Q6ICC9",
  "gene_name": "Retrotransposon Gag-like protein 6",
  "term_id": "UNKNOWN:0003",
  "term_label": "Unknown cellular component"
}